{
  "gene": "UniProtKB:A0A0U1RRN3",
  "term_id": "UNKNOWN:0001",
  "gene_symbol": "MISFA",
  "term_label": "Unknown molecular function",
  "gene_name": "Mitochondrial sheath formation-associated protein"
}